regulation of mRNA catabolic process [GO:0061013] (biological process) Relationships: is a type of GO:0009894; is a type of GO:0010468; is a type of GO:1903311; regulates GO:0006402 Sources: GOC:ascb_2009, GOC:dph, GOC:tb Also known as: regulation of mRNA decay Definition: Any process that modulates the rate, frequency, or extent of a mRNA catabolic process, the chemical reactions and pathways resulting in the breakdown of RNA, ribonucleic acid, one of the two main type of nucleic acid, consisting of a long, unbranched macromolecule formed from ribonucleotides joined in 3',5'-phosphodiester linkage. Subtypes: regulation of mRNA stability [GO:0043488], regulation of nuclear-transcribed mRNA poly(A) tail shortening [GO:0060211], positive regulation of mRNA catabolic process [GO:0061014], GO:0106288, regulation of nuclear mRNA surveillance of meiosis-specific transcripts [GO:0120270], negative regulation of mRNA catabolic process [GO:1902373], regulation of mitochondrial mRNA catabolic process [GO:1905637], regulation of nuclear-transcribed mRNA catabolic process, nonsense-mediated decay [GO:2000622]